protein K27-linked deubiquitination [GO:1990167] (biological process) References: PMID:23827681 Definition: A protein deubiquitination process in which a K27-linked ubiquitin chain, i.e. a polymer of ubiquitin formed by linkages between lysine residues at position 27 of the ubiquitin monomers, is removed from a protein. Relationships: is a type of protein deubiquitination [GO:0016579]